{
  "term_id": "UNKNOWN:0002",
  "gene": "UniProtKB:Q16342",
  "gene_name": "Programmed cell death protein 2",
  "gene_symbol": "PDCD2",
  "term_label": "Unknown biological process"
}